regulation of sterol transport [GO:0032371] (biological process) Definition: Any process that modulates the frequency, rate or extent of the directed movement of sterols into, out of or within a cell, or between cells, by means of some agent such as a transporter or pore. Sources: GOC:mah Relationships: is a type of GO:0032368; regulates sterol transport [GO:0015918] Subtypes: negative regulation of sterol transport [GO:0032372], positive regulation of sterol transport [GO:0032373], GO:0032374, regulation of intracellular sterol transport [GO:0032380], regulation of sterol import [GO:2000909]